{
  "gene": "UniProtKB:O95428",
  "gene_name": "Papilin",
  "term_id": "UNKNOWN:0001",
  "term_label": "Unknown molecular function",
  "gene_symbol": "PAPLN"
}